{
  "term_id": "UNKNOWN:0002",
  "gene_symbol": "OR4C12",
  "term_label": "Unknown biological process",
  "gene": "UniProtKB:Q96R67",
  "gene_name": "Olfactory receptor 4C12"
}